{
  "gene_name": "Calpain-5",
  "term_id": "GO:0005737",
  "term_label": "cytoplasm",
  "gene_symbol": "CAPN5",
  "gene": "UniProtKB:O15484"
}